{
  "term_id": "UNKNOWN:0002",
  "gene": "UniProtKB:P0DX00",
  "term_label": "Unknown biological process",
  "gene_symbol": "GOLGA6L24",
  "gene_name": "Golgin subfamily A member 6-like protein 24"
}